{
  "gene": "UniProtKB:Q9ULL0",
  "gene_name": "Acrosomal protein KIAA1210",
  "term_label": "Unknown biological process",
  "gene_symbol": "KIAA1210",
  "term_id": "UNKNOWN:0002"
}